{
  "gene_name": "Serine protease FAM111B",
  "term_id": "GO:0106300",
  "term_label": "protein-DNA covalent cross-linking repair",
  "gene": "UniProtKB:Q6SJ93",
  "gene_symbol": "FAM111B"
}